{
  "gene_symbol": "OR5M10",
  "gene_name": "Olfactory receptor 5M10",
  "term_id": "UNKNOWN:0003",
  "term_label": "Unknown cellular component",
  "gene": "UniProtKB:Q6IEU7"
}